trochlear nerve maturation [GO:0021640] (biological process) Definition: A developmental process, independent of morphogenetic (shape) change, that is required for the trochlear nerve to attain its fully functional state. The trochlear nerve is a motor nerve and is the only cranial nerve to exit the brain dorsally. The trochlear nerve innervates the superior oblique muscle. Sources: GOC:cls, GOC:dgh, GOC:dph, GOC:jid, GO_REF:0000021 Also known as: CN IV maturation Relationships: is a type of cranial nerve maturation [GO:0021605]; is part of trochlear nerve development [GO:0021558]